{
  "term_label": "intracellular potassium ion homeostasis",
  "gene_name": "Potassium-transporting ATPase alpha chain 1",
  "term_id": "GO:0030007",
  "gene_symbol": "ATP4A",
  "gene": "UniProtKB:P20648"
}